{
  "term_label": "Unknown biological process",
  "term_id": "UNKNOWN:0002",
  "gene_name": "Olfactory receptor 4D2",
  "gene": "UniProtKB:P58180",
  "gene_symbol": "OR4D2"
}